{
  "term_label": "site of double-strand break",
  "gene": "UniProtKB:Q9UBZ9",
  "term_id": "GO:0035861",
  "gene_name": "DNA repair protein REV1",
  "gene_symbol": "REV1"
}